{
  "gene_name": "Histone H3-like centromeric protein A",
  "term_id": "GO:0030527",
  "gene": "UniProtKB:P49450",
  "gene_symbol": "CENPA",
  "term_label": "structural constituent of chromatin"
}